aerobic respiration, using arsenite as electron donor [GO:0043554] (biological process) Relationships: is a type of aerobic respiration [GO:0009060]; is a type of GO:0015975 Sources: GOC:mlg Definition: The oxidation of arsenite to arsenate, using oxygen (O2) as the electron acceptor. Arsenite oxidase provides electrons to an electron carrier which transfers them to oxygen utilizing respiratory systems.